{
  "gene_name": "Cadherin-7",
  "gene": "UniProtKB:Q9ULB5",
  "term_id": "GO:0016477",
  "term_label": "cell migration",
  "gene_symbol": "CDH7"
}